cytoskeletal protein binding [GO:0008092] (molecular function) Definition: Binding to a protein component of a cytoskeleton (actin, microtubule, or intermediate filament cytoskeleton). Relationships: is a type of protein binding [GO:0005515] Sources: GOC:mah Subtypes: actin binding [GO:0003779], cytoskeletal regulatory protein binding [GO:0005519], GO:0005523, GO:0015631, myosin binding [GO:0017022], GO:0017166, kinesin binding [GO:0019894], troponin C binding [GO:0030172], ankyrin binding [GO:0030506], spectrin binding [GO:0030507], filamin binding [GO:0031005], troponin I binding [GO:0031013], troponin T binding [GO:0031014], titin binding [GO:0031432], GO:0031433, dynactin binding [GO:0034452], GO:0042805, tau protein binding [GO:0048156], FATZ binding [GO:0051373], GO:1990147